{
  "term_label": "post-translational protein targeting to membrane, translocation",
  "gene_symbol": "SEC61A2",
  "gene_name": "Protein transport protein Sec61 subunit alpha isoform 2",
  "term_id": "GO:0031204",
  "gene": "UniProtKB:Q9H9S3"
}